{
  "gene_name": "Uncharacterized protein C11orf87",
  "gene_symbol": "C11orf87",
  "term_label": "Unknown biological process",
  "gene": "UniProtKB:Q6NUJ2",
  "term_id": "UNKNOWN:0002"
}